{
  "gene": "UniProtKB:Q01118",
  "term_id": "GO:0005248",
  "term_label": "voltage-gated sodium channel activity",
  "gene_name": "Sodium channel protein type 7 subunit alpha",
  "gene_symbol": "SCN7A"
}